{
  "gene_name": "Anthrax toxin receptor-like",
  "gene": "UniProtKB:A6NF34",
  "gene_symbol": "ANTXRL",
  "term_id": "GO:0009986",
  "term_label": "cell surface"
}